{
  "gene_symbol": "TRBV16",
  "term_label": "Unknown molecular function",
  "gene_name": "T cell receptor beta variable 16",
  "gene": "UniProtKB:A0A087WV62",
  "term_id": "UNKNOWN:0001"
}